regulation of mating projection assembly [GO:0031383] (BP) Definition: Any process that modulates the frequency, rate, or extent of mating projection formation by unicellular fungi. Also known as: regulation of mating projection biogenesis Relationships: is a type of regulation of developmental process [GO:0050793]; is a type of regulation of plasma membrane bounded cell projection assembly [GO:0120032]; regulates GO:0031382 References: PMID:14734532 Subtypes: regulation of initiation of mating projection growth [GO:0031384], regulation of termination of mating projection growth [GO:0031385], positive regulation of mating projection assembly [GO:1902917]